{
  "gene_name": "Glutamate receptor ionotropic, kainate 3",
  "gene": "UniProtKB:Q13003",
  "gene_symbol": "GRIK3",
  "term_label": "postsynaptic density membrane",
  "term_id": "GO:0098839"
}